{
  "gene": "UniProtKB:Q96DN0",
  "gene_name": "Endoplasmic reticulum resident protein 27",
  "term_id": "GO:0006457",
  "term_label": "protein folding",
  "gene_symbol": "ERP27"
}